{
  "gene_name": "P3 protein",
  "term_id": "GO:0008508",
  "gene_symbol": "SLC10A3",
  "gene": "UniProtKB:P09131",
  "term_label": "bile acid:sodium symporter activity"
}